{
  "term_label": "serine-type peptidase activity",
  "gene_symbol": "TMPRSS11F",
  "gene": "UniProtKB:Q6ZWK6",
  "term_id": "GO:0008236",
  "gene_name": "Transmembrane protease serine 11F"
}